{
  "gene": "UniProtKB:Q96SB3",
  "gene_name": "Neurabin-2",
  "term_label": "actin filament organization",
  "term_id": "GO:0007015",
  "gene_symbol": "PPP1R9B"
}